{
  "gene_symbol": "NSF",
  "term_id": "GO:0043001",
  "term_label": "Golgi to plasma membrane protein transport",
  "gene_name": "Vesicle-fusing ATPase",
  "gene": "UniProtKB:P46459"
}